{
  "gene": "UniProtKB:Q15714",
  "gene_name": "TSC22 domain family protein 1",
  "term_id": "GO:0005634",
  "term_label": "nucleus",
  "gene_symbol": "TSC22D1"
}